{
  "gene_symbol": "UBE3D",
  "term_label": "protein polyubiquitination",
  "term_id": "GO:0000209",
  "gene_name": "E3 ubiquitin-protein ligase E3D",
  "gene": "UniProtKB:Q7Z6J8"
}